{
  "gene_symbol": "PAQR5",
  "term_id": "UNKNOWN:0002",
  "gene": "UniProtKB:Q9NXK6",
  "gene_name": "Membrane progestin receptor gamma",
  "term_label": "Unknown biological process"
}